{
  "term_id": "GO:0008200",
  "term_label": "ion channel inhibitor activity",
  "gene_symbol": "STOML1",
  "gene_name": "Stomatin-like protein 1",
  "gene": "UniProtKB:Q9UBI4"
}